{
  "term_id": "UNKNOWN:0001",
  "term_label": "Unknown molecular function",
  "gene_name": "Armadillo repeat-containing protein 1",
  "gene": "UniProtKB:Q9NVT9",
  "gene_symbol": "ARMC1"
}